{
  "gene": "UniProtKB:Q8NGJ8",
  "gene_symbol": "OR51S1",
  "term_label": "plasma membrane",
  "term_id": "GO:0005886",
  "gene_name": "Olfactory receptor 51S1"
}